{
  "gene_symbol": "ADGRE3",
  "gene": "UniProtKB:Q9BY15",
  "term_id": "GO:0005886",
  "gene_name": "Adhesion G protein-coupled receptor E3",
  "term_label": "plasma membrane"
}